anterior midgut development [GO:0007496] (biological process) Definition: The process whose specific outcome is the progression of the anterior midgut over time, from its formation to the mature structure. Sources: GOC:jid Relationships: is a type of anatomical structure development [GO:0048856]; is part of midgut development [GO:0007494]